{
  "gene_symbol": "OR4F16",
  "term_label": "Unknown biological process",
  "gene_name": "Olfactory receptor 4F3_4F16_4F29",
  "gene": "UniProtKB:Q6IEY1",
  "term_id": "UNKNOWN:0002"
}